{
  "gene": "UniProtKB:Q6IPT4",
  "gene_symbol": "CYB5RL",
  "term_id": "UNKNOWN:0003",
  "gene_name": "NADH-cytochrome b5 reductase-like",
  "term_label": "Unknown cellular component"
}